{
  "term_id": "GO:0006357",
  "gene_name": "Bromodomain-containing protein 4",
  "term_label": "regulation of transcription by RNA polymerase II",
  "gene": "UniProtKB:O60885",
  "gene_symbol": "BRD4"
}